{
  "gene_name": "PHD finger protein 11",
  "term_id": "UNKNOWN:0002",
  "gene": "UniProtKB:Q9UIL8",
  "term_label": "Unknown biological process",
  "gene_symbol": "PHF11"
}